I-kappaB/NF-kappaB complex [GO:0033256] (cellular component) Definition: A protein complex containing an inhibitory-kappaB (I-kappaB/IKB) protein and one or more copies of an NF-kappaB protein. In the resting state, NF-kappaB dimers are bound to I-kappaB proteins, sequestering NF-kappaB in the cytoplasm. References: PMID:9407099 Sources: GOC:bf, GOC:mah Subtypes: Bcl3/NF-kappaB2 complex [GO:0033257] Relationships: is a type of intracellular protein-containing complex [GO:0140535]